{
  "term_label": "adaptive thermogenesis",
  "gene_name": "Putative mitochondrial transporter UCP3",
  "term_id": "GO:1990845",
  "gene": "UniProtKB:P55916",
  "gene_symbol": "UCP3"
}